L-phenylalanine N-monooxygenase activity [GO:0102684] (molecular function) Sources: EC:1.14.14.40, GOC:pz Relationships: is a type of oxidoreductase activity, acting on paired donors, with incorporation or reduction of molecular oxygen, NAD(P)H as one donor, and incorporation of one atom of oxygen [GO:0016709] Definition: Catalysis of the reaction: L-phenylalanine + 2 NADPH + 2 O2 + 2 H+ = (E)-phenylacetaldehyde oxime + 2 NADP + 3 H2O + carbon dioxide.